{
  "gene_name": "Kinesin-like protein KIF20B",
  "gene_symbol": "KIF20B",
  "term_id": "GO:0005737",
  "gene": "UniProtKB:Q96Q89",
  "term_label": "cytoplasm"
}